root hair elongation [GO:0048767] (biological process) Regulation: regulated by regulation of root hair elongation [GO:1902890]; negatively regulated by GO:1902891; positively regulated by positive regulation of root hair elongation [GO:1902892] References: PMID:12468740 Sources: GOC:jid Relationships: is a type of developmental cell growth [GO:0048588]; is_a GO:0060560; is part of root hair cell development [GO:0080147] Definition: The process in which the root hair grows longer.